{
  "term_label": "Golgi cisterna membrane",
  "gene_name": "Golgin subfamily A member 8H",
  "gene": "UniProtKB:P0CJ92",
  "term_id": "GO:0032580",
  "gene_symbol": "GOLGA8H"
}